{
  "gene": "UniProtKB:Q9BXL7",
  "term_id": "GO:0043123",
  "term_label": "positive regulation of canonical NF-kappaB signal transduction",
  "gene_symbol": "CARD11",
  "gene_name": "Caspase recruitment domain-containing protein 11"
}